{
  "gene_symbol": "IL5",
  "gene": "UniProtKB:P05113",
  "term_id": "GO:0005125",
  "gene_name": "Interleukin-5",
  "term_label": "cytokine activity"
}